biological_process [GO:0008150] (biological process) Note: Note that, in addition to forming the root of the biological process ontology, this term is recommended for the annotation of gene products whose biological process is unknown. When this term is used for annotation, it indicates that no information was available about the biological process of the gene product annotated as of the date the annotation was made; the evidence code 'no data' (ND), is used to indicate this. Also known as: biological process, physiological process, single organism process, single-organism process Sources: GOC:pdt Definition: A biological process is the execution of a genetically-encoded biological module or program. It consists of all the steps required to achieve the specific biological objective of the module. A biological process is accomplished by a particular set of molecular functions carried out by specific gene products (or macromolecular complexes), often in a highly regulated manner and in a particular temporal sequence. Subtypes: immune system process [GO:0002376], cellular process [GO:0009987], viral process [GO:0016032], GO:0022414, multicellular organismal process [GO:0032501], developmental process [GO:0032502], GO:0040007, locomotion [GO:0040011], homeostatic process [GO:0042592], GO:0043473, biological process involved in interspecies interaction between organisms [GO:0044419], biological phase [GO:0044848], rhythmic process [GO:0048511], response to stimulus [GO:0050896], localization [GO:0051179], biological process involved in intraspecies interaction between organisms [GO:0051703], biological regulation [GO:0065007], detoxification [GO:0098754] Regulation: positively regulated by positive regulation of biological process [GO:0048518]; negatively regulated by negative regulation of biological process [GO:0048519]; regulated by regulation of biological process [GO:0050789]